{
  "term_id": "GO:0005005",
  "term_label": "transmembrane-ephrin receptor activity",
  "gene": "UniProtKB:O15197",
  "gene_name": "Ephrin type-B receptor 6",
  "gene_symbol": "EPHB6"
}